{
  "term_label": "Unknown biological process",
  "gene_name": "B-cell CLL_lymphoma 7 protein family member C",
  "gene_symbol": "BCL7C",
  "term_id": "UNKNOWN:0002",
  "gene": "UniProtKB:Q8WUZ0"
}